{
  "term_label": "cytosol",
  "gene_symbol": "OPLAH",
  "gene": "UniProtKB:O14841",
  "term_id": "GO:0005829",
  "gene_name": "5-oxoprolinase"
}